Wnt receptor internalization [GO:0038017] (BP) Also known as: Wnt receptor endocytosis Definition: A receptor-mediated endocytosis process that results in the movement of a Wnt receptor from the plasma membrane to the inside of the cell. Relationships: is a type of receptor internalization [GO:0031623] References: PMID:17908284 Sources: GOC:bf